putrescine biosynthetic process [GO:0009446] (biological process) Definition: The chemical reactions and pathways resulting in the formation of putrescine, 1,4-diaminobutane; putrescine can be synthesized from arginine or ornithine and is the metabolic precursor of spermidine and spermine. Sources: GOC:go_curators, ISBN:0198506732 Also known as: putrescine anabolism, putrescine biosynthesis, putrescine formation, putrescine synthesis Relationships: is a type of polyamine biosynthetic process [GO:0006596]; is_a putrescine metabolic process [GO:0009445] Subtypes: putrescine biosynthetic process from arginine [GO:0033388]